{
  "term_id": "UNKNOWN:0001",
  "gene_symbol": "TATDN2",
  "gene_name": "Putative deoxyribonuclease TATDN2",
  "gene": "UniProtKB:Q93075",
  "term_label": "Unknown molecular function"
}